{
  "term_id": "GO:1902387",
  "gene": "UniProtKB:Q96JA3",
  "gene_symbol": "PLEKHA8",
  "gene_name": "Pleckstrin homology domain-containing family A member 8",
  "term_label": "ceramide 1-phosphate binding"
}